{
  "term_label": "cytokine activity",
  "term_id": "GO:0005125",
  "gene_name": "Lymphotoxin-beta",
  "gene": "UniProtKB:Q06643",
  "gene_symbol": "LTB"
}